{
  "gene_symbol": "ZNF774",
  "gene_name": "Zinc finger protein 774",
  "gene": "UniProtKB:Q6NX45",
  "term_id": "GO:0000981",
  "term_label": "DNA-binding transcription factor activity, RNA polymerase II-specific"
}